oxidized pyrimidine DNA binding [GO:0032358] (molecular function) Sources: GOC:vk Definition: Binding to a DNA region containing an oxidized pyrimidine residue. Also known as: oxidised pyrimidine DNA binding, oxidized pyrimidine base DNA binding, oxidized pyrimidine nucleobase DNA binding Relationships: is a type of GO:0032356